{
  "gene_name": "RNA-binding motif protein, Y chromosome, family 1 member D",
  "term_label": "mRNA binding",
  "gene_symbol": "RBMY1D",
  "gene": "UniProtKB:P0C7P1",
  "term_id": "GO:0003729"
}